{
  "gene": "UniProtKB:Q8N1F8",
  "term_id": "GO:0140311",
  "term_label": "protein sequestering activity",
  "gene_symbol": "STK11IP",
  "gene_name": "Serine_threonine-protein kinase 11-interacting protein"
}